{
  "gene_name": "Single-minded homolog 2",
  "gene": "UniProtKB:Q14190",
  "term_id": "GO:0006357",
  "term_label": "regulation of transcription by RNA polymerase II",
  "gene_symbol": "SIM2"
}